{
  "gene_name": "Importin-11",
  "term_id": "GO:0006606",
  "gene_symbol": "IPO11",
  "term_label": "protein import into nucleus",
  "gene": "UniProtKB:Q9UI26"
}